{
  "gene": "UniProtKB:Q8N8Z8",
  "gene_symbol": "ZNF441",
  "gene_name": "Zinc finger protein 441",
  "term_label": "nucleus",
  "term_id": "GO:0005634"
}